{
  "gene_symbol": "OLFML1",
  "gene_name": "Olfactomedin-like protein 1",
  "gene": "UniProtKB:Q6UWY5",
  "term_label": "Unknown molecular function",
  "term_id": "UNKNOWN:0001"
}